{
  "gene": "UniProtKB:G9CGD6",
  "term_id": "GO:0030674",
  "term_label": "protein-macromolecule adaptor activity",
  "gene_name": "CNK3_IPCEF1 fusion protein",
  "gene_symbol": "CNK3/IPCEF1"
}